{
  "term_label": "microtubule cytoskeleton organization",
  "term_id": "GO:0000226",
  "gene_name": "Cingulin",
  "gene": "UniProtKB:Q9P2M7",
  "gene_symbol": "CGN"
}